{
  "gene_symbol": "MYO7A",
  "term_label": "endocytosis",
  "gene_name": "Unconventional myosin-VIIa",
  "term_id": "GO:0006897",
  "gene": "UniProtKB:Q13402"
}